{
  "term_id": "UNKNOWN:0002",
  "gene_name": "Tetratricopeptide repeat protein 9C",
  "gene": "UniProtKB:Q8N5M4",
  "gene_symbol": "TTC9C",
  "term_label": "Unknown biological process"
}